protein K29-linked ubiquitination [GO:0035519] (biological process) References: PMID:17028573 Relationships: is a type of GO:0000209 Definition: A protein ubiquitination process in which a polymer of ubiquitin, formed by linkages between lysine residues at position 29 of the ubiquitin monomers, is added to a protein. K29-linked ubiquitination targets the substrate protein for degradation. Also known as: protein K29-linked polyubiquitination